{
  "gene": "UniProtKB:Q13702",
  "term_id": "GO:0005886",
  "gene_name": "43 kDa receptor-associated protein of the synapse",
  "gene_symbol": "RAPSN",
  "term_label": "plasma membrane"
}